{
  "gene_symbol": "GMFB",
  "gene": "UniProtKB:P60983",
  "term_id": "GO:0071846",
  "term_label": "actin filament debranching",
  "gene_name": "Glia maturation factor beta"
}